{
  "term_label": "tropomyosin binding",
  "term_id": "GO:0005523",
  "gene": "UniProtKB:P13805",
  "gene_symbol": "TNNT1",
  "gene_name": "Troponin T, slow skeletal muscle"
}